{
  "gene_symbol": "RB1CC1",
  "gene": "UniProtKB:Q8TDY2",
  "term_id": "GO:0034727",
  "gene_name": "RB1-inducible coiled-coil protein 1",
  "term_label": "piecemeal microautophagy of the nucleus"
}